regulation of chondrocyte differentiation [GO:0032330] (biological process) Subtypes: negative regulation of chondrocyte differentiation [GO:0032331], positive regulation of chondrocyte differentiation [GO:0032332], GO:0061181, GO:1902738 Relationships: is_a regulation of cell differentiation [GO:0045595]; is a type of regulation of cartilage development [GO:0061035]; regulates chondrocyte differentiation [GO:0002062] Definition: Any process that modulates the frequency, rate or extent of chondrocyte differentiation. Sources: GOC:mah